negative regulation of cellotriose catabolic process [GO:2000937] (biological process) Relationships: is a type of negative regulation of catabolic process [GO:0009895]; is a type of negative regulation of carbohydrate metabolic process [GO:0045912]; is a type of regulation of cellotriose catabolic process [GO:2000936]; negatively regulates cellotriose catabolic process [GO:2000894] Sources: GOC:mengo_curators Definition: Any process that stops, prevents or reduces the frequency, rate or extent of cellotriose catabolic process. Also known as: negative regulation of cellotriose catabolism